histone H3K deacetylase activity [GO:0141050] (molecular function) Subtypes: histone H3K14 deacetylase activity, hydrolytic mechanism [GO:0031078], histone H3K14 deacetylase activity, NAD-dependent [GO:0032041], histone H3K9 deacetylase activity, hydrolytic mechanism [GO:0032129], histone H3K9 deacetylase activity, NAD-dependent [GO:0046969], histone H3K18 deacetylase activity, NAD-dependent [GO:0097372], histone H3K56 deacetylase activity, NAD-dependent [GO:0140765], histone H3K4 deacetylase activity, NAD-dependent [GO:0141222], GO:1990162 Definition: Removal of an acetyl group from a lysine residue in a histone H3. Relationships: is_a histone deacetylase activity [GO:0004407] References: PMID:9893272 Sources: GOC:pg Note: Histone deacytylase (HDAC) enzymes are divided into four classes: the Class I Rpd3-like proteins (in human: HDAC1, HDAC2, HDAC3, and HDAC8); the Class II Hda1-like proteins (in human: HDAC4, HDAC5, HDAC6, HDAC7, HDAC9, and HDAC10); the Class III Sir2-like proteins (in human: SIRT1, SIRT2, SIRT3, SIRT4, SIRT5, SIRT6, and SIRT7); and the Class IV protein (HDAC11 in human). Except for Class III enzymes, the mechanism is a metal-dependent hydrolysis of the acetylated substrate. The Class III HDACs use NAD+ as a reactant to deacetylate acetyl lysine residues of protein substrates forming nicotinamide, the deacetylated product, and the metabolite 2'-O-acetyl-ADP-ribose. Therefore, Class III are classified as transferases (EC:2) and others are hydrolases (EC:3).